{
  "term_label": "odorant binding",
  "gene_name": "Olfactory receptor 5F1",
  "term_id": "GO:0005549",
  "gene": "UniProtKB:O95221",
  "gene_symbol": "OR5F1"
}